{
  "gene_name": "Deoxyuridine 5'-triphosphate nucleotidohydrolase, mitochondrial",
  "gene_symbol": "DUT",
  "term_label": "magnesium ion binding",
  "gene": "UniProtKB:P33316",
  "term_id": "GO:0000287"
}